Las1 complex [GO:0090730] (cellular component) References: PMID:26638174 Sources: GOC:vw Also known as: Las1-Grc3-Rat1-Rai1 Relationships: is a type of GO:1902555; is a type of protein kinase complex [GO:1902911]; is a type of exoribonuclease complex [GO:1905354]; is part of GO:0005829 Definition: A four subunit complex, that comprises all the necessary RNA processing enzymes (endonuclease, polynucleotide kinase, and exonuclease) to mediate 'cistronic rRNA transcript ITS2 (internal transcribed spacer) cleavage' (GO:0000448).